{
  "gene": "UniProtKB:Q86XR7",
  "gene_symbol": "TICAM2",
  "gene_name": "TIR domain-containing adapter molecule 2",
  "term_label": "signaling adaptor activity",
  "term_id": "GO:0035591"
}